{
  "term_label": "zinc ion binding",
  "term_id": "GO:0008270",
  "gene_symbol": "GCH1",
  "gene": "UniProtKB:P30793",
  "gene_name": "GTP cyclohydrolase 1"
}